extracellular ligand-gated monoatomic ion channel activity [GO:0005230] (molecular function) Relationships: is a type of GO:0015276 Sources: GOC:mtg_transport, ISBN:0815340729 Definition: Enables the transmembrane transfer of an ion by a channel that opens when a specific extracellular ligand has been bound by the channel complex or one of its constituent parts. Subtypes: excitatory extracellular ligand-gated monoatomic ion channel activity [GO:0005231], inhibitory extracellular ligand-gated monoatomic ion channel activity [GO:0005237], transmitter-gated monoatomic ion channel activity [GO:0022824], extracellular ammonia-gated monoatomic ion channel activity [GO:0036081], extracellular phenylacetaldehyde-gated monoatomic ion channel activity [GO:0036082] Also known as: extracellular ligand-gated ion channel activity